{
  "gene_symbol": "RASGEF1C",
  "gene": "UniProtKB:Q8N431",
  "term_label": "plasma membrane",
  "term_id": "GO:0005886",
  "gene_name": "Ras-GEF domain-containing family member 1C"
}